{
  "gene_name": "Serine_threonine-protein kinase MRCK gamma",
  "term_label": "protein serine/threonine kinase activity",
  "term_id": "GO:0004674",
  "gene": "UniProtKB:Q6DT37",
  "gene_symbol": "CDC42BPG"
}